male germline stem cell symmetric division [GO:0098730] (BP) Definition: The symmetric division of a male germline stem cell to produce two male germline stem cells. An example of this is found in mammalian spermatogonial stem cells, some proportion of which divide symmetrically, so amplifying the population. The choice between asymmetric and symmetric division in this case appears to be internal and stochastic. Relationships: is a type of GO:0098729 References: PMID:19948499 Sources: GOC:dos